{
  "term_id": "UNKNOWN:0001",
  "gene": "UniProtKB:Q99674",
  "gene_name": "Cell growth regulator with EF hand domain protein 1",
  "gene_symbol": "CGREF1",
  "term_label": "Unknown molecular function"
}